{
  "term_id": "GO:0004351",
  "gene": "UniProtKB:Q99259",
  "gene_symbol": "GAD1",
  "term_label": "glutamate decarboxylase activity",
  "gene_name": "Glutamate decarboxylase 1"
}